{
  "term_label": "GTP binding",
  "gene_symbol": "RAB26",
  "gene_name": "Ras-related protein Rab-26",
  "gene": "UniProtKB:Q9ULW5",
  "term_id": "GO:0005525"
}